regulation of orcinol biosynthetic process [GO:1900701] (biological process) Subtypes: negative regulation of orcinol biosynthetic process [GO:1900702], positive regulation of orcinol biosynthetic process [GO:1900703] Also known as: regulation of orcinol anabolism, regulation of orcinol biosynthesis, regulation of orcinol formation, regulation of orcinol synthesis Sources: GOC:TermGenie, GOC:di Definition: Any process that modulates the frequency, rate or extent of orcinol biosynthetic process. Relationships: is a type of regulation of secondary metabolite biosynthetic process [GO:1900376]; regulates orcinol biosynthetic process [GO:0046197]